{
  "gene_symbol": "KIFAP3",
  "gene": "UniProtKB:Q92845",
  "gene_name": "Kinesin-associated protein 3",
  "term_id": "GO:0007018",
  "term_label": "microtubule-based movement"
}